{
  "term_id": "GO:0003714",
  "gene_name": "DNA-binding protein inhibitor ID-3",
  "term_label": "transcription corepressor activity",
  "gene_symbol": "ID3",
  "gene": "UniProtKB:Q02535"
}